{
  "term_label": "intracellular calcium ion homeostasis",
  "gene_name": "Mitochondrial sodium_calcium exchanger protein",
  "gene_symbol": "SLC8B1",
  "gene": "UniProtKB:Q6J4K2",
  "term_id": "GO:0006874"
}